{
  "gene": "UniProtKB:Q6IMI6",
  "term_label": "sulfation",
  "gene_symbol": "SULT1C3",
  "term_id": "GO:0051923",
  "gene_name": "Sulfotransferase 1C3"
}